{
  "term_label": "nucleosomal DNA binding",
  "gene": "UniProtKB:P16403",
  "term_id": "GO:0031492",
  "gene_name": "Histone H1.2",
  "gene_symbol": "H1-2"
}